dolichyl-phosphate beta-glucosyltransferase activity [GO:0004581] (molecular function) Definition: Catalysis of the reaction: UDP-glucose + dolichyl phosphate = UDP + dolichyl beta-D-glucosyl phosphate. Also known as: UDP-glucose dolichyl-phosphate glucosyltransferase activity, UDP-glucose:dolichol phosphate glucosyltransferase activity, UDP-glucose:dolicholphosphoryl glucosyltransferase activity, UDP-glucose:dolichyl monophosphate glucosyltransferase activity, UDP-glucose:dolichyl phosphate glucosyltransferase activity, UDP-glucose:dolichyl-phosphate beta-D-glucosyltransferase activity, UDPglucose:dolichyl-phosphate beta-D-glucosyltransferase activity, polyprenyl phosphate:UDP-D-glucose glucosyltransferase activity, uridine diphosphoglucose-dolichol glucosyltransferase activity Relationships: is a type of UDP-glucosyltransferase activity [GO:0035251] Sources: EC:2.4.1.117